{
  "gene_name": "Homeobox protein Hox-A5",
  "term_id": "GO:0005634",
  "gene": "UniProtKB:P20719",
  "term_label": "nucleus",
  "gene_symbol": "HOXA5"
}